{
  "gene_name": "Zinc finger CCHC domain-containing protein 7",
  "term_id": "GO:0003723",
  "gene": "UniProtKB:Q8N3Z6",
  "gene_symbol": "ZCCHC7",
  "term_label": "RNA binding"
}